4-hydroxy-L-threonine aldolase activity [GO:0103042] (molecular function) Sources: GOC:pz, RHEA:28779 Relationships: is a type of aldehyde-lyase activity [GO:0016832] Definition: Catalysis of the reaction: 4-hydroxy-L-threonine = glycolaldehyde + glycine.